{
  "gene_name": "Melanoma-associated antigen B17",
  "term_id": "GO:0005634",
  "term_label": "nucleus",
  "gene_symbol": "MAGEB17",
  "gene": "UniProtKB:A8MXT2"
}